{
  "gene_name": "Serine protease HTRA4",
  "gene_symbol": "HTRA4",
  "term_id": "GO:0004252",
  "gene": "UniProtKB:P83105",
  "term_label": "serine-type endopeptidase activity"
}